{
  "term_label": "sphingolipid metabolic process",
  "gene_name": "Protein ARV1",
  "gene_symbol": "ARV1",
  "gene": "UniProtKB:Q9H2C2",
  "term_id": "GO:0006665"
}